{
  "term_id": "GO:0006270",
  "term_label": "DNA replication initiation",
  "gene_name": "Cell division control protein 6 homolog",
  "gene": "UniProtKB:Q99741",
  "gene_symbol": "CDC6"
}